{
  "term_label": "extracellular space",
  "gene_symbol": "ORM1",
  "gene_name": "Alpha-1-acid glycoprotein 1",
  "term_id": "GO:0005615",
  "gene": "UniProtKB:P02763"
}